{
  "gene_symbol": "GTPBP10",
  "term_label": "Unknown biological process",
  "gene_name": "GTP-binding protein 10",
  "term_id": "UNKNOWN:0002",
  "gene": "UniProtKB:A4D1E9"
}